{
  "gene": "UniProtKB:Q2M3W8",
  "gene_symbol": "ZNF181",
  "term_id": "GO:0000978",
  "term_label": "RNA polymerase II cis-regulatory region sequence-specific DNA binding",
  "gene_name": "Zinc finger protein 181"
}